pancreatic E cell fate commitment [GO:0090106] (biological process) Relationships: is_a cell fate commitment [GO:0045165]; is part of pancreatic epsilon cell differentiation [GO:0090104] Definition: The commitment of a cell to a pancreatic E cell fate and its capacity to differentiate into a pancreatic E cell. Sources: GOC:dph, GOC:tb